{
  "gene_symbol": "TENM1",
  "term_label": "protein homodimerization activity",
  "term_id": "GO:0042803",
  "gene_name": "Teneurin-1",
  "gene": "UniProtKB:Q9UKZ4"
}